{
  "gene": "UniProtKB:Q9HAV4",
  "gene_name": "Exportin-5",
  "term_id": "GO:0005737",
  "gene_symbol": "XPO5",
  "term_label": "cytoplasm"
}